negative regulation of cholesterol biosynthetic process [GO:0045541] (biological process) Relationships: is_a regulation of cholesterol biosynthetic process [GO:0045540]; is_a negative regulation of cholesterol metabolic process [GO:0090206]; is a type of negative regulation of sterol biosynthetic process [GO:0106119]; is a type of GO:1902931; negatively regulates cholesterol biosynthetic process [GO:0006695] Definition: Any process that stops, prevents, or reduces the frequency, rate or extent of the chemical reactions and pathways resulting in the formation of cholesterol. Sources: GOC:go_curators Also known as: down regulation of cholesterol biosynthetic process, down-regulation of cholesterol biosynthetic process, downregulation of cholesterol biosynthetic process, negative regulation of cholesterol anabolism, negative regulation of cholesterol biosynthesis, negative regulation of cholesterol formation, negative regulation of cholesterol synthesis, inhibition of cholesterol biosynthetic process